regulation of exocytic insertion of neurotransmitter receptor to postsynaptic membrane [GO:0099145] (biological process) Definition: Any process that modulates the frequency, rate or extent of exocytic fusion of neurotransmitter receptor containing vesicles into the postsynaptic membrane. Sources: GOC:dos Relationships: is a type of GO:0017157; is a type of GO:0051223; is a type of regulation of biological quality [GO:0065008]; is a type of regulation of receptor localization to synapse [GO:1902683]; is a type of regulation of protein localization to cell periphery [GO:1904375]; is a type of regulation of protein localization to membrane [GO:1905475]; RO_0002211 exocytic insertion of neurotransmitter receptor to postsynaptic membrane [GO:0098967]